secondary cell wall [GO:0009531] (cellular component) Relationships: is a type of plant-type cell wall [GO:0009505] Sources: GOC:jid, ISBN:0943088399 Definition: A plant cell wall that is no longer able to expand and so does not permit growth. Secondary cell walls contain less pectin that primary cell walls. The secondary cell is mostly composed of cellulose and is strengthened with lignin.